{
  "term_label": "proteasome regulatory particle, base subcomplex",
  "gene_symbol": "PSMC3",
  "gene_name": "26S proteasome regulatory subunit 6A",
  "term_id": "GO:0008540",
  "gene": "UniProtKB:P17980"
}